{
  "term_id": "GO:0061630",
  "gene_symbol": "RNF40",
  "gene_name": "E3 ubiquitin-protein ligase BRE1B",
  "gene": "UniProtKB:O75150",
  "term_label": "ubiquitin protein ligase activity"
}